reproductive system development [GO:0061458] (biological process) Sources: GOC:dph Definition: The progression of the reproductive system over time from its formation to the mature structure. The reproductive system consists of the organs that function in reproduction. Relationships: is_a system development [GO:0048731] Subtypes: male genitalia development [GO:0030539]